{
  "gene_name": "Dysbindin domain-containing protein 1",
  "term_label": "regulation of signal transduction",
  "gene_symbol": "DBNDD1",
  "gene": "UniProtKB:Q9H9R9",
  "term_id": "GO:0009966"
}